{
  "gene_name": "Lipid transferase CIDEB",
  "term_label": "lipid droplet",
  "gene": "UniProtKB:Q9UHD4",
  "gene_symbol": "CIDEB",
  "term_id": "GO:0005811"
}